bilobe structure assembly [GO:0140528] (biological process) Also known as: bilobe structure biogenesis, bilobe structure formation, kinetoplastid flagellar hook complex assembly Definition: The assembly and organization of a bilobe structure, a cytoskeletal structure in some kinetoplastid species linking the structures of the ciliary pocket collar and the flagellum attachment zone (aka cilium attachment zone). References: PMID:18443217, PMID:32675283 Relationships: is a type of cellular component assembly [GO:0022607]; is part of GO:0007010